{
  "term_label": "gamma-aminobutyric acid signaling pathway",
  "gene": "UniProtKB:Q16445",
  "term_id": "GO:0007214",
  "gene_symbol": "GABRA6",
  "gene_name": "Gamma-aminobutyric acid receptor subunit alpha-6"
}